regulation of Roundabout signaling pathway [GO:0035386] (biological process) Relationships: is a type of GO:0009966; RO_0002211 GO:0035385 Also known as: regulation of Roundabout signalling pathway Subtypes: GO:0035387, positive regulation of Roundabout signaling pathway [GO:0035388] Definition: Any process that modulates the frequency, rate or extent of the Roundabout signaling pathway. Sources: GOC:BHF